nitrate reductase (NADPH) activity [GO:0050464] (molecular function) Sources: RHEA:19061 Definition: Catalysis of the reaction: nitrite + NADP+ + H2O = nitrate + NADPH + H+. Relationships: is a type of nitrate reductase [NAD(P)H] activity [GO:0050463] Also known as: assimilatory nitrate reductase activity, NADPH-nitrate reductase activity, NADPH:nitrate oxidoreductase activity, NADPH:nitrate reductase activity, assimilatory NADPH-nitrate reductase activity, assimilatory reduced nicotinamide adenine dinucleotide phosphate-nitrate reductase activity, nitrate reductase (NADPH(2)) activity, nitrate reductase (NADPH2), nitrite:NADP+ oxidoreductase activity, triphosphopyridine nucleotide-nitrate reductase activity